{
  "gene_symbol": "ITGB6",
  "gene_name": "Integrin beta-6",
  "gene": "UniProtKB:P18564",
  "term_label": "focal adhesion",
  "term_id": "GO:0005925"
}